{
  "gene_name": "Ras-related protein Rab-5A",
  "gene_symbol": "RAB5A",
  "term_label": "endocytosis",
  "gene": "UniProtKB:P20339",
  "term_id": "GO:0006897"
}